{
  "gene_name": "Myopalladin",
  "gene": "UniProtKB:Q86TC9",
  "term_label": "plasma membrane",
  "term_id": "GO:0005886",
  "gene_symbol": "MYPN"
}